{
  "term_label": "cell surface",
  "gene_name": "Integrin alpha-6",
  "gene": "UniProtKB:P23229",
  "gene_symbol": "ITGA6",
  "term_id": "GO:0009986"
}